{
  "term_id": "GO:0140374",
  "gene": "UniProtKB:P09914",
  "gene_symbol": "IFIT1",
  "term_label": "antiviral innate immune response",
  "gene_name": "Interferon-induced protein with tetratricopeptide repeats 1"
}